{
  "term_id": "GO:0032580",
  "gene_symbol": "GOLGA6A",
  "gene_name": "Golgin subfamily A member 6A",
  "term_label": "Golgi cisterna membrane",
  "gene": "UniProtKB:Q9NYA3"
}